{
  "gene_name": "Hepatocyte growth factor-regulated tyrosine kinase substrate",
  "gene_symbol": "HGS",
  "term_label": "ubiquitin binding",
  "gene": "UniProtKB:O14964",
  "term_id": "GO:0043130"
}